{
  "gene_symbol": "PI4KA",
  "term_id": "GO:0004430",
  "term_label": "1-phosphatidylinositol 4-kinase activity",
  "gene": "UniProtKB:P42356",
  "gene_name": "Phosphatidylinositol 4-kinase alpha"
}